DNA nucleotidylexotransferase activity [GO:0003912] (molecular function) Sources: EC:2.7.7.31 Definition: Catalysis of the reaction: deoxynucleoside triphosphate + DNA(n) = diphosphate + DNA(n+1); template-independent extension of the 3'-end of a DNA strand by one nucleotide at a time. Relationships: is_a GO:0034061 Also known as: TdT, addase activity, deoxynucleotidyl terminal transferase activity, deoxyribonucleic acid nucleotidyltransferase activity, deoxyribonucleic nucleotidyltransferase activity, nucleoside-triphosphate:DNA deoxynucleotidylexotransferase activity, terminal addition enzyme activity, terminal deoxynucleotide transferase activity, terminal deoxynucleotidyltransferase activity, terminal deoxyribonucleotidyltransferase activity, terminal transferase activity